synaptic vesicle, readily releasable pool [GO:1990474] (cellular component) Also known as: readily releasable pool of synaptic vesicles, RRP References: PMID:22745285 Sources: GOC:pad Relationships: is a type of synaptic vesicle [GO:0008021]; is part of terminal bouton [GO:0043195] Definition: A synaptic vesicle belonging to the pool of vesicles that are the first to be released as a result of chemical or electrical stimulation e.g. by an action potential, have the highest presynaptic membrane fusion probability and correspond to about 1% of the total number of synaptic vesicles at a resting terminal bouton.